{
  "term_id": "GO:0007195",
  "gene_symbol": "DRD3",
  "term_label": "adenylate cyclase-inhibiting dopamine receptor signaling pathway",
  "gene": "UniProtKB:P35462",
  "gene_name": "D(3) dopamine receptor"
}